{
  "term_label": "U12 snRNA binding",
  "gene_name": "RNA-binding protein 41",
  "gene_symbol": "RBM41",
  "term_id": "GO:0030626",
  "gene": "UniProtKB:Q96IZ5"
}